syncytial blastoderm mitotic cell cycle [GO:0035186] (biological process) Definition: Mitotic division cycles 10 to 13 of the insect embryo. This is the second phase of the syncytial period where nuclei divide in a common cytoplasm without cytokinesis. The majority of migrating nuclei reach the embryo surface during cycle 10, after which they divide less synchronously than before, and the syncytial blastoderm cycles lengthen progressively. Sources: ISBN:0879694238 Relationships: is a type of cell cycle comprising mitosis without cytokinesis [GO:0033301]; is a type of GO:0045448 Regulation: regulated by regulation of syncytial blastoderm mitotic cell cycle [GO:0007348]; negatively regulated by GO:0046003; positively regulated by positive regulation of syncytial blastoderm mitotic cell cycle [GO:0046004]